negative regulation of pectin catabolic process [GO:2001004] (biological process) Definition: Any process that stops, prevents or reduces the frequency, rate or extent of pectin catabolic process. Relationships: is a type of negative regulation of catabolic process [GO:0009895]; is a type of GO:0010605; is a type of negative regulation of carbohydrate metabolic process [GO:0045912]; is a type of GO:2001003; RO_0002212 pectin catabolic process [GO:0045490] Also known as: negative regulation of pectin breakdown, negative regulation of pectin catabolism, negative regulation of pectin degradation Sources: GOC:mengo_curators